{
  "term_label": "nucleocytoplasmic transport",
  "gene_symbol": "ANP32A",
  "gene_name": "Acidic leucine-rich nuclear phosphoprotein 32 family member A",
  "gene": "UniProtKB:P39687",
  "term_id": "GO:0006913"
}